{
  "gene_symbol": "DCAF1",
  "term_label": "histone H2AT120 kinase activity",
  "term_id": "GO:1990244",
  "gene": "UniProtKB:Q9Y4B6",
  "gene_name": "DDB1- and CUL4-associated factor 1"
}